urotensin II receptor activity [GO:0001604] (molecular function) Definition: Combining with urotensin II to initiate a change in cell activity. Relationships: is a type of GO:0008528 References: PMID:15102493 Sources: GOC:mah